alkene binding [GO:0072328] (molecular function) Subtypes: GO:0051740 Relationships: is_a small molecule binding [GO:0036094] Definition: Binding to an alkene, any acyclic branched or unbranched hydrocarbon having one carbon-carbon double bond and the general formula CnH2n. Sources: GOC:mah